{
  "gene_name": "Alpha-synuclein",
  "gene": "UniProtKB:P37840",
  "term_id": "GO:0043025",
  "gene_symbol": "SNCA",
  "term_label": "neuronal cell body"
}